regulation of heart contraction [GO:0008016] (biological process) Relationships: is a type of GO:1903522; regulates heart contraction [GO:0060047] Subtypes: GO:0002026, regulation of heart rate [GO:0002027], regulation of heart contraction involved in acute-phase response [GO:0002531], negative regulation of heart contraction [GO:0045822], positive regulation of heart contraction [GO:0045823], GO:0055117, cardiac conduction [GO:0061337], regulation of cardiac conduction [GO:1903779] Sources: GOC:dph, GOC:go_curators, GOC:tb Also known as: regulation of cardiac contraction Definition: Any process that modulates the frequency, rate or extent of heart contraction. Heart contraction is the process in which the heart decreases in volume in a characteristic way to propel blood through the body.